{
  "term_label": "phosphatidylinositol-4,5-bisphosphate binding",
  "gene_symbol": "VIL1",
  "gene": "UniProtKB:P09327",
  "gene_name": "Villin-1",
  "term_id": "GO:0005546"
}